{
  "gene": "UniProtKB:Q86X60",
  "term_label": "Unknown molecular function",
  "gene_symbol": "FAM72B",
  "gene_name": "Protein FAM72B",
  "term_id": "UNKNOWN:0001"
}